{
  "term_id": "GO:0007342",
  "term_label": "fusion of sperm to egg plasma membrane involved in single fertilization",
  "gene": "UniProtKB:A6ND01",
  "gene_symbol": "IZUMO1R",
  "gene_name": "Sperm-egg fusion protein Juno"
}